{
  "term_label": "deacetylase activity",
  "gene_symbol": "NDST1",
  "gene_name": "Bifunctional heparan sulfate N-deacetylase_N-sulfotransferase 1",
  "gene": "UniProtKB:P52848",
  "term_id": "GO:0019213"
}